{
  "gene_name": "Zymogen granule protein 16 homolog B",
  "gene_symbol": "ZG16B",
  "gene": "UniProtKB:Q96DA0",
  "term_id": "UNKNOWN:0002",
  "term_label": "Unknown biological process"
}